ventricular compact myocardium morphogenesis [GO:0003223] (biological process) Subtypes: left ventricular compact myocardium morphogenesis [GO:0003224], GO:0003226 Relationships: is a type of ventricular cardiac muscle tissue morphogenesis [GO:0055010] Sources: GOC:mtg_heart Definition: The process in which the anatomical structures of the compact cardiac ventricle muscle are generated and organized.